{
  "gene_symbol": "RNF133",
  "gene_name": "E3 ubiquitin-protein ligase RNF133",
  "gene": "UniProtKB:Q8WVZ7",
  "term_id": "GO:0005794",
  "term_label": "Golgi apparatus"
}